{
  "term_id": "GO:0036503",
  "gene_symbol": "FBXO17",
  "term_label": "ERAD pathway",
  "gene": "UniProtKB:Q96EF6",
  "gene_name": "F-box only protein 17"
}